{
  "term_id": "GO:0016045",
  "gene_name": "NLR family CARD domain-containing protein 4",
  "term_label": "detection of bacterium",
  "gene": "UniProtKB:Q9NPP4",
  "gene_symbol": "NLRC4"
}